{
  "gene_name": "Voltage-dependent calcium channel gamma-3 subunit",
  "term_label": "postsynaptic density membrane",
  "term_id": "GO:0098839",
  "gene_symbol": "CACNG3",
  "gene": "UniProtKB:O60359"
}